{
  "term_id": "GO:0005886",
  "gene_name": "T cell receptor beta variable 3-1",
  "term_label": "plasma membrane",
  "gene": "UniProtKB:A0A576",
  "gene_symbol": "TRBV3-1"
}